{
  "gene_name": "Serine protease inhibitor Kazal-type 9",
  "gene_symbol": "SPINK9",
  "term_id": "GO:0045861",
  "term_label": "negative regulation of proteolysis",
  "gene": "UniProtKB:Q5DT21"
}